{
  "term_id": "UNKNOWN:0003",
  "gene": "UniProtKB:Q8N1G0",
  "gene_symbol": "ZNF687",
  "term_label": "Unknown cellular component",
  "gene_name": "Zinc finger protein 687"
}